{
  "gene": "UniProtKB:P10645",
  "term_id": "GO:0033604",
  "term_label": "negative regulation of catecholamine secretion",
  "gene_name": "Chromogranin-A",
  "gene_symbol": "CHGA"
}